{
  "gene_symbol": "IGHV4OR15-8",
  "gene_name": "Immunoglobulin heavy variable 4_OR15-8 (non-functional) (Fragment)",
  "term_id": "GO:0016064",
  "term_label": "immunoglobulin mediated immune response",
  "gene": "UniProtKB:A0A075B7B6"
}